{
  "gene": "UniProtKB:Q9BQE9",
  "term_label": "Unknown molecular function",
  "term_id": "UNKNOWN:0001",
  "gene_symbol": "BCL7B",
  "gene_name": "B-cell CLL_lymphoma 7 protein family member B"
}